{
  "term_label": "extracellular space",
  "gene_name": "Protein Wnt-3a",
  "term_id": "GO:0005615",
  "gene_symbol": "WNT3A",
  "gene": "UniProtKB:P56704"
}